{
  "gene_symbol": "BCAT1",
  "gene_name": "Branched-chain-amino-acid aminotransferase, cytosolic",
  "gene": "UniProtKB:P54687",
  "term_label": "L-valine biosynthetic process",
  "term_id": "GO:0009099"
}